{
  "gene": "UniProtKB:Q96IV0",
  "gene_symbol": "NGLY1",
  "term_id": "GO:0005634",
  "gene_name": "Peptide-N(4)-(N-acetyl-beta-glucosaminyl)asparagine amidase",
  "term_label": "nucleus"
}